{
  "gene_name": "Proteasome subunit beta type-5",
  "gene": "UniProtKB:P28074",
  "term_id": "GO:0005634",
  "gene_symbol": "PSMB5",
  "term_label": "nucleus"
}